{
  "term_id": "GO:0008210",
  "gene_name": "UDP-glucuronosyltransferase 1A8",
  "gene_symbol": "UGT1A8",
  "term_label": "estrogen metabolic process",
  "gene": "UniProtKB:Q9HAW9"
}